negative regulation of Golgi vesicle fusion to target membrane [GO:0048216] (biological process) Definition: Any process that stops, prevents, or reduces the frequency, rate or extent of Golgi vesicle fusion to target membrane. References: PMID:10219233 Sources: GOC:jid, ISBN:0716731363 Also known as: down regulation of Golgi vesicle fusion to target membrane, down-regulation of Golgi vesicle fusion to target membrane, downregulation of Golgi vesicle fusion to target membrane, inhibition of Golgi vesicle fusion to target membrane Relationships: is a type of GO:0031339; is a type of regulation of Golgi vesicle fusion to target membrane [GO:0048214]; negatively regulates GO:0048210